{
  "gene": "UniProtKB:Q9BSG5",
  "term_label": "signaling receptor activity",
  "term_id": "GO:0038023",
  "gene_name": "Retbindin",
  "gene_symbol": "RTBDN"
}